transmembrane transporter complex [GO:1902495] (cellular component) Relationships: is a type of GO:0098796; is a type of transporter complex [GO:1990351] Definition: A transmembrane protein complex which enables the transfer of a substance from one side of a membrane to the other. References: PMID:18024586 Sources: GOC:TermGenie, GOC:bhm Subtypes: cytochrome o ubiquinol oxidase complex [GO:0009319], protein-N(PI)-phosphohistidine-sugar phosphotransferase complex [GO:0009357], high-affinity iron permease complex [GO:0033573], monoatomic ion channel complex [GO:0034702], respiratory chain complex I [GO:0045271], GO:0045275, respiratory chain complex IV [GO:0045277], high-affinity iron exporter complex [GO:0061841], calcium:proton antiporter complex [GO:0061993], curli secretion complex [GO:0062155], ATPase dependent transmembrane transport complex [GO:0098533], ammonium transmembrane transporter complex [GO:0110067], methionine-importing complex [GO:1902509], potassium:proton antiporter complex [GO:1903103], copper ion transmembrane transporter complex [GO:1903113], silver ion transmembrane transporter complex [GO:1903114], macrolide transmembrane transporter complex [GO:1990195], MdtBC Complex [GO:1990203], EmrE multidrug transporter complex [GO:1990207], efflux pump complex [GO:1990281], GO:1990662, GO:7770001